{
  "gene_symbol": "GPR15",
  "term_label": "G protein-coupled receptor signaling pathway",
  "gene_name": "G-protein coupled receptor 15",
  "gene": "UniProtKB:P49685",
  "term_id": "GO:0007186"
}